{
  "gene": "UniProtKB:P28300",
  "term_id": "GO:0031012",
  "gene_symbol": "LOX",
  "term_label": "extracellular matrix",
  "gene_name": "Protein-lysine 6-oxidase"
}